cytoplasm protein quality control [GO:0140455] (biological process) References: PMID:32075773 Definition: The chemical reactions and pathways resulting in the breakdown of misfolded proteins in the cytoplasm, which are either targeted to cytoplasmic proteasomes for degradation or protected by chaperones to shield thermosensitive proteins from degradation until conditions allow disaggregation and refolding. Relationships: is a type of protein quality control for misfolded or incompletely synthesized proteins [GO:0006515] Subtypes: cytoplasm protein quality control by the ubiquitin-proteasome system [GO:0071629]